{
  "term_label": "UMP biosynthetic process",
  "term_id": "GO:0006222",
  "gene_symbol": "UMPS",
  "gene": "UniProtKB:P11172",
  "gene_name": "Uridine 5'-monophosphate synthase"
}